Edg-2 lysophosphatidic acid receptor binding [GO:0031755] (molecular function) Sources: GOC:mah, GOC:nln Also known as: LPA1 receptor binding, Edg-2 lysophosphatidic acid receptor ligand Definition: Binding to an Edg-2 lysophosphatidic acid receptor. Relationships: is a type of endothelial differentiation G protein-coupled receptor binding [GO:0031753]